{
  "gene": "UniProtKB:O14921",
  "gene_symbol": "RGS13",
  "term_id": "GO:0045744",
  "term_label": "negative regulation of G protein-coupled receptor signaling pathway",
  "gene_name": "Regulator of G-protein signaling 13"
}